positive regulation of phospholipase C-activating G protein-coupled receptor signaling pathway [GO:1900738] (biological process) Definition: Any process that activates or increases the frequency, rate or extent of phospholipase C-activating G protein-coupled receptor signaling pathway. Also known as: activation of G protein signaling, coupled to IP3 second messenger (phospholipase C activating), activation of G protein signalling, coupled to IP3 second messenger (phospholipase C activating), activation of G-protein coupled receptor signaling pathway coupled to IP3 second messenger, activation of G-protein signaling, coupled to IP3 second messenger (phospholipase C activating), activation of G-protein signalling, coupled to IP3 second messenger (phospholipase C activating), activation of PLC-activating GPCR signaling pathway, positive regulation of G protein signaling, coupled to IP3 second messenger (phospholipase C activating), positive regulation of G protein signalling, coupled to IP3 second messenger (phospholipase C activating), positive regulation of G-protein coupled receptor signaling pathway coupled to IP3 second messenger, positive regulation of G-protein signaling, coupled to IP3 second messenger (phospholipase C activating), positive regulation of G-protein signalling, coupled to IP3 second messenger (phospholipase C activating), positive regulation of PLC-activating GPCR signaling pathway, positive regulation of phospholipase C-activating G-protein coupled receptor signaling pathway, up regulation of G protein signaling, coupled to IP3 second messenger (phospholipase C activating), up regulation of G protein signalling, coupled to IP3 second messenger (phospholipase C activating), up regulation of G-protein coupled receptor signaling pathway coupled to IP3 second messenger, up regulation of G-protein signaling, coupled to IP3 second messenger (phospholipase C activating), up regulation of G-protein signalling, coupled to IP3 second messenger (phospholipase C activating), up regulation of PLC-activating GPCR signaling pathway, up regulation of phospholipase C-activating G-protein coupled receptor signaling pathway, up-regulation of G protein signaling, coupled to IP3 second messenger (phospholipase C activating), up-regulation of G protein signalling, coupled to IP3 second messenger (phospholipase C activating), up-regulation of G-protein coupled receptor signaling pathway coupled to IP3 second messenger, up-regulation of G-protein signaling, coupled to IP3 second messenger (phospholipase C activating), up-regulation of G-protein signalling, coupled to IP3 second messenger (phospholipase C activating), up-regulation of PLC-activating GPCR signaling pathway, up-regulation of phospholipase C-activating G-protein coupled receptor signaling pathway, upregulation of G protein signaling, coupled to IP3 second messenger (phospholipase C activating), upregulation of G protein signalling, coupled to IP3 second messenger (phospholipase C activating), upregulation of G-protein coupled receptor signaling pathway coupled to IP3 second messenger, upregulation of G-protein signaling, coupled to IP3 second messenger (phospholipase C activating), upregulation of G-protein signalling, coupled to IP3 second messenger (phospholipase C activating), upregulation of PLC-activating GPCR signaling pathway, upregulation of phospholipase C-activating G-protein coupled receptor signaling pathway, activation of phospholipase C-activating G-protein coupled receptor signaling pathway, activation of phospholipase C-activating dopamine receptor signaling pathway, positive regulation of phospholipase C-activating dopamine receptor signaling pathway, up regulation of phospholipase C-activating dopamine receptor signaling pathway, up-regulation of phospholipase C-activating dopamine receptor signaling pathway, upregulation of phospholipase C-activating dopamine receptor signaling pathway, activation of activation of phospholipase C activity by G-protein coupled receptor protein signaling pathway coupled to IP3 second messenger, positive regulation of activation of phospholipase C activity by G-protein coupled receptor protein signaling pathway coupled to IP3 second messenger, up regulation of activation of phospholipase C activity by G-protein coupled receptor protein signaling pathway coupled to IP3 second messenger, up-regulation of activation of phospholipase C activity by G-protein coupled receptor protein signaling pathway coupled to IP3 second messenger, upregulation of activation of phospholipase C activity by G-protein coupled receptor protein signaling pathway coupled to IP3 second messenger Relationships: is a type of positive regulation of G protein-coupled receptor signaling pathway [GO:0045745]; is a type of GO:1900736; positively regulates GO:0007200 Sources: GOC:BHF, GOC:TermGenie